S-adenosylmethionine biosynthetic process [GO:0006556] (biological process) Relationships: is a type of sulfur compound biosynthetic process [GO:0044272]; is a type of S-adenosylmethionine metabolic process [GO:0046500] Also known as: S-adenosyl methionine biosynthesis, S-adenosyl methionine biosynthetic process, S-adenosylmethionine anabolism, S-adenosylmethionine biosynthesis, S-adenosylmethionine formation, S-adenosylmethionine synthesis, SAM biosynthetic process Sources: GOC:go_curators, ISBN:0198506732 Definition: The chemical reactions and pathways resulting in the formation of S-adenosylmethionine, S-(5'-adenosyl)-L-methionine, an important intermediate in one-carbon metabolism.